beta 2 integrin biosynthetic process [GO:0045114] (biological process) Regulation: regulated by regulation of beta 2 integrin biosynthetic process [GO:0045115]; negatively regulated by negative regulation of beta 2 integrin biosynthetic process [GO:0045774]; positively regulated by GO:0045775 Sources: GOC:go_curators Also known as: beta 2 integrin anabolism, beta 2 integrin biosynthesis, beta 2 integrin formation, beta 2 integrin synthesis Relationships: is a type of GO:0045112 Definition: The chemical reactions and pathways resulting in the formation of beta 2 integrins, a subfamily of integrins which contain the beta 2 subunit.